{
  "term_label": "Unknown cellular component",
  "gene_name": "Zinc finger protein 234",
  "gene": "UniProtKB:Q14588",
  "term_id": "UNKNOWN:0003",
  "gene_symbol": "ZNF234"
}